{
  "gene": "UniProtKB:P58304",
  "gene_name": "Visual system homeobox 2",
  "term_id": "GO:1990837",
  "term_label": "sequence-specific double-stranded DNA binding",
  "gene_symbol": "VSX2"
}